regulation of ribosomal protein gene transcription by RNA polymerase II [GO:0060962] (biological process) Sources: GOC:dph, GOC:tb, GOC:txnOH Also known as: regulation of ribosomal protein gene transcription from RNA polymerase II promoter Definition: Any process that modulates the frequency, rate or extent of the synthesis of RNA from ribosomal protein genes mediated by RNA polymerase II. Relationships: is a type of GO:0006357 Subtypes: GO:0010688, positive regulation of ribosomal protein gene transcription by RNA polymerase II [GO:0060963]